regulation of glial cell-derived neurotrophic factor production [GO:1900166] (biological process) Subtypes: negative regulation of glial cell-derived neurotrophic factor production [GO:1900167], GO:1900168 Definition: Any process that modulates the frequency, rate or extent of glial cell-derived neurotrophic factor production. Also known as: regulation of GDNF secretion, regulation of glial cell-derived neurotrophic factor secretion, regulation of glial cell line-derived neurotrophic factor secretion Sources: GOC:TermGenie, GOC:yaf Relationships: is a type of GO:0001817; RO_0002211 glial cell-derived neurotrophic factor production [GO:0044467]